interleukin-19 binding [GO:0042013] (molecular function) Definition: Binding to interleukin-19. Relationships: is a type of cytokine binding [GO:0019955] Also known as: IL-19 binding Sources: GOC:jl